{
  "term_id": "GO:0045087",
  "gene": "UniProtKB:Q99836",
  "gene_symbol": "MYD88",
  "term_label": "innate immune response",
  "gene_name": "Myeloid differentiation primary response protein MyD88"
}